{
  "term_id": "GO:0043410",
  "gene_name": "Fibroblast growth factor 3",
  "term_label": "positive regulation of MAPK cascade",
  "gene_symbol": "FGF3",
  "gene": "UniProtKB:P11487"
}